{
  "gene_symbol": "GIT1",
  "term_label": "cytosol",
  "gene": "UniProtKB:Q9Y2X7",
  "gene_name": "ARF GTPase-activating protein GIT1",
  "term_id": "GO:0005829"
}